{
  "gene_symbol": "OR51H1",
  "gene": "UniProtKB:Q8NH63",
  "term_label": "Unknown biological process",
  "gene_name": "Olfactory receptor 51H1",
  "term_id": "UNKNOWN:0002"
}